female analia development [GO:0045497] (biological process) Definition: The process whose specific outcome is the progression of the analia of the female over time, from formation to the mature structure. The analia is the posterior-most vertral appendage that develops from the genital disc. An example of this process is found in Drosophila melanogaster. References: PMID:11494318 Sources: GOC:mtg_sensu Relationships: is a type of analia development [GO:0007487]